{
  "gene_name": "Serine_threonine-protein kinase MRCK beta",
  "term_label": "protein serine/threonine kinase activity",
  "term_id": "GO:0004674",
  "gene_symbol": "CDC42BPB",
  "gene": "UniProtKB:Q9Y5S2"
}